{
  "term_id": "GO:0005254",
  "gene_name": "Glycine receptor subunit alpha-2",
  "gene": "UniProtKB:P23416",
  "term_label": "chloride channel activity",
  "gene_symbol": "GLRA2"
}